{
  "gene_name": "B-cell CLL_lymphoma 6 member B protein",
  "term_label": "DNA-binding transcription repressor activity, RNA polymerase II-specific",
  "term_id": "GO:0001227",
  "gene": "UniProtKB:Q8N143",
  "gene_symbol": "BCL6B"
}